latent virus replication [GO:0019045] (biological process) Sources: ISBN:0781702534 Definition: Any process required for latent viral replication in a cell. Relationships: is_a viral process [GO:0016032]; is part of viral latency [GO:0019042]